RNA polymerase II CTD heptapeptide repeat kinase activity [GO:0008353] (molecular function) Subtypes: RNA polymerase II CTD heptapeptide repeat Y1 kinase activity [GO:0140833], RNA polymerase II CTD heptapeptide repeat S2 kinase activity [GO:0140834], RNA polymerase II CTD heptapeptide repeat T4 kinase activity [GO:0140835], RNA polymerase II CTD heptapeptide repeat S5 kinase activity [GO:0140836], RNA polymerase II CTD heptapeptide repeat S7 kinase activity [GO:0140837] References: PMID:28248323 Sources: EC:2.7.11.23, GOC:mah Definition: Catalysis of the reaction: ATP + RNA polymerase II large subunit CTD heptapeptide repeat (consensus YSPTSPS) = ADP + H+ + phosphorylated RNA polymerase II. Relationships: is a type of protein serine/threonine kinase activity [GO:0004674]; is a type of GO:0140994 Also known as: RNA polymerase subunit kinase activity, RNA-polymerase-subunit kinase activity, [RNA-polymerase]-subunit kinase activity, RNA polymerase II carboxy-terminal domain kinase activity, CTD kinase activity